{
  "gene_symbol": "EVI2A",
  "term_label": "Unknown biological process",
  "term_id": "UNKNOWN:0002",
  "gene": "UniProtKB:P22794",
  "gene_name": "Protein EVI2A"
}